S-adenosyl-L-methionine transmembrane transporter activity [GO:0000095] (molecular function) Subtypes: S-adenosyl-L-methionine:S-adenosyl-L-homocysteine antiporter activity [GO:0180003] Relationships: is a type of sulfur compound transmembrane transporter activity [GO:1901682]; is part of S-adenosyl-L-methionine transmembrane transport [GO:1901962] Definition: Enables the transfer of S-adenosylmethionine from one side of a membrane to the other. S-adenosylmethionine is S-(5'-adenosyl)-L-methionine, an important intermediate in one-carbon metabolism. Also known as: S-adenosylmethionine transporter activity, S-adenosyl methionine permease activity, S-adenosyl methionine transporter activity, S-adenosylmethionine permease activity, S-adenosylmethionine transmembrane transporter activity, SAM transmembrane transporter activity Sources: GOC:ai